anthocyanin 5-O-glucosyltransferase activity [GO:0080018] (molecular function) Definition: Catalysis of the reaction: an anthocyanin + UDP-D-glucose = an anthocyanin-5-O-glucoside + UDP. Relationships: is a type of UDP-glucosyltransferase activity [GO:0035251] References: PMID:15807784